AMP phosphorylation [GO:0006756] (biological process) Sources: GOC:ai Definition: The process of introducing a phosphate group into AMP, adenosine monophosphate, to produce ADP. Addition of two phosphate groups produces ATP. Relationships: is a type of ATP biosynthetic process [GO:0006754]; is a type of AMP metabolic process [GO:0046033]; is a type of nucleoside monophosphate phosphorylation [GO:0046940]